{
  "term_label": "receptor tyrosine kinase binding",
  "gene": "UniProtKB:Q06124",
  "gene_name": "Tyrosine-protein phosphatase non-receptor type 11",
  "gene_symbol": "PTPN11",
  "term_id": "GO:0030971"
}